hepatocyte cell migration [GO:0002194] (biological process) Definition: The orderly movement of a hepatocyte during the development of the liver. Hepatocytes emerge from the hepatic epithelium, populating the septum transversum and lateral mesenchymal areas of the hepatic lobes. References: PMID:9794819 Sources: CL:0000182 Relationships: is a type of cell migration [GO:0016477]